symbiont-mediated cell-to-cell migration by invasive hypha [GO:0140649] (biological process) Relationships: is a type of symbiont-mediated cell-to-cell migration in host [GO:0106259] Also known as: host tissue colonization, invasive growth, plant tissue colonization, cell-to-cell migration by invasive hypha, invasive hyphae formation Definition: The directional movement of a hyphal filament from one host cell to another. This process involves the clearance of plant-derived plasmodesmal occlusion materials, cytoskeleton based constriction of invasive hypha to traverse plasmodesmata. Septins and F-actin are reorganized into an hourglass shape at the point of maximum hyphal constriction. Note: Do not confuse with ' GO:0036267 invasive filamentous growth ', which doesn't include invasion of cells within the host. References: PMID:29567712